{
  "gene_symbol": "RORA",
  "term_label": "RNA polymerase II cis-regulatory region sequence-specific DNA binding",
  "gene": "UniProtKB:P35398",
  "term_id": "GO:0000978",
  "gene_name": "Nuclear receptor ROR-alpha"
}